peptidyl-lysine crotonylation [GO:0140066] (biological process) Relationships: is a type of protein acylation [GO:0043543] References: PMID:25818647 Sources: Wikipedia:crotonyl Definition: The crotonylation of a lysine residue in a protein. Crotonyl is the univalent radical CH3-CH=CH-CO- derived from crotonic acid. Regulation: RO_0002211 by regulation of peptidyl-lysine crotonylation [GO:0120093]; RO_0002212 by negative regulation of peptidyl-lysine crotonylation [GO:0120094]